{
  "gene_symbol": "OR4F6",
  "term_label": "olfactory receptor activity",
  "gene_name": "Olfactory receptor 4F6",
  "gene": "UniProtKB:Q8NGB9",
  "term_id": "GO:0004984"
}